{
  "term_label": "RNA polymerase II, core complex",
  "gene_name": "DNA-directed RNA polymerases I, II, and III subunit RPABC1",
  "gene": "UniProtKB:P19388",
  "term_id": "GO:0005665",
  "gene_symbol": "POLR2E"
}